nuclear telomere cap complex [GO:0000783] (cellular component) Subtypes: shelterin complex [GO:0070187], CST complex [GO:1990879] Note: Note that this term can be used in place of the obsolete cellular component term 'telomere ; GO:0005696'. Use with caution because this term refers to a specific protein complex and not a region of the chromosome. Relationships: is a type of telomere cap complex [GO:0000782]; is a type of nuclear protein-containing complex [GO:0140513] Definition: A complex of DNA and protein located at the end of a linear chromosome in the nucleus that protects and stabilizes a linear chromosome. Sources: GOC:elh